{
  "term_label": "plasma membrane",
  "term_id": "GO:0005886",
  "gene": "UniProtKB:P78357",
  "gene_symbol": "CNTNAP1",
  "gene_name": "Contactin-associated protein 1"
}